{
  "term_label": "DNA replication",
  "gene_name": "Treslin",
  "gene_symbol": "TICRR",
  "term_id": "GO:0006260",
  "gene": "UniProtKB:Q7Z2Z1"
}